{
  "term_id": "GO:0000127",
  "gene_symbol": "GTF3C2",
  "gene_name": "General transcription factor 3C polypeptide 2",
  "term_label": "transcription factor TFIIIC complex",
  "gene": "UniProtKB:Q8WUA4"
}